{
  "term_label": "cytokine activity",
  "term_id": "GO:0005125",
  "gene": "UniProtKB:P43026",
  "gene_name": "Growth_differentiation factor 5",
  "gene_symbol": "GDF5"
}